heptadecane metabolic process [GO:1900635] (biological process) Relationships: is a type of hydrocarbon metabolic process [GO:0120252] Subtypes: heptadecane biosynthetic process [GO:1900636] Also known as: heptadecane metabolism Sources: GOC:TermGenie, GOC:mengo_curators Definition: The chemical reactions and pathways involving heptadecane.